{
  "gene": "UniProtKB:Q92889",
  "gene_name": "DNA repair endonuclease XPF",
  "gene_symbol": "ERCC4",
  "term_id": "GO:0000014",
  "term_label": "single-stranded DNA endodeoxyribonuclease activity"
}